{
  "term_label": "Unknown cellular component",
  "gene_symbol": "DEFB112",
  "term_id": "UNKNOWN:0003",
  "gene": "UniProtKB:Q30KQ8",
  "gene_name": "Beta-defensin 112"
}